{
  "gene_name": "Neuromodulin",
  "gene_symbol": "GAP43",
  "gene": "UniProtKB:P17677",
  "term_id": "GO:0035727",
  "term_label": "lysophosphatidic acid binding"
}